{
  "gene_name": "Mesothelin-like protein",
  "term_label": "Unknown molecular function",
  "gene_symbol": "MSLNL",
  "gene": "UniProtKB:Q96KJ4",
  "term_id": "UNKNOWN:0001"
}